{
  "term_id": "GO:0046513",
  "gene_name": "Serine palmitoyltransferase small subunit A",
  "gene_symbol": "SPTSSA",
  "term_label": "ceramide biosynthetic process",
  "gene": "UniProtKB:Q969W0"
}